{
  "gene": "UniProtKB:Q8IVJ8",
  "gene_name": "APRG1 tumor suppressor candidate",
  "term_label": "Unknown molecular function",
  "term_id": "UNKNOWN:0001",
  "gene_symbol": "APRG1"
}